negative regulation of growth plate cartilage chondrocyte proliferation [GO:0061914] (biological process) Definition: Any process that decreases the rate, frequency, or extent of the multiplication or reproduction of chondrocytes in a growing endochondral bone, resulting in the expansion of a cell population. Relationships: is a type of GO:0003420; is a type of negative regulation of cell population proliferation [GO:0008285]; is a type of GO:0046621; negatively regulates GO:0003419 References: PMID:19264869